{
  "term_label": "protein-lysine-acetyltransferase activity",
  "gene": "UniProtKB:Q5FWF5",
  "gene_symbol": "ESCO1",
  "term_id": "GO:0061733",
  "gene_name": "N-acetyltransferase ESCO1"
}